{
  "term_id": "GO:0004558",
  "gene_name": "Sucrase-isomaltase, intestinal",
  "gene": "UniProtKB:P14410",
  "term_label": "alpha-1,4-glucosidase activity",
  "gene_symbol": "SI"
}